{
  "term_label": "Unknown molecular function",
  "gene": "UniProtKB:P01597",
  "gene_name": "Immunoglobulin kappa variable 1-39",
  "term_id": "UNKNOWN:0001",
  "gene_symbol": "IGKV1-39"
}